beta-catenin-TCF complex assembly [GO:1904837] (biological process) Relationships: is a type of protein-containing complex assembly [GO:0065003] Definition: The aggregation, arrangement and bonding together of a set of components to form a beta-catenin-TCF complex. References: PMID:18936100 Sources: GOC:PARL, GOC:TermGenie, GOC:bf, GO_REF:0000079 Regulation: regulated by regulation of beta-catenin-TCF complex assembly [GO:1904863]; negatively regulated by GO:1904864; positively regulated by positive regulation of beta-catenin-TCF complex assembly [GO:1904865] Also known as: beta-catenin-TCF complex formation, beta-catenin/LEF complex assembly, beta-catenin/LEF complex formation, beta-catenin/T-cell factor complex assembly, beta-catenin/T-cell factor complex formation, beta-catenin/lymphoid enhancer binding factor complex assembly, beta-catenin/lymphoid enhancer binding factor complex formation